{
  "term_id": "GO:0000813",
  "term_label": "ESCRT I complex",
  "gene_name": "Vacuolar protein sorting-associated protein 28 homolog",
  "gene_symbol": "VPS28",
  "gene": "UniProtKB:Q9UK41"
}